microtubule plus-end binding [GO:0051010] (molecular function) Relationships: is a type of microtubule binding [GO:0008017] Definition: Binding to the plus end of a microtubule. References: PMID:14557818, PMID:14614826 Sources: GOC:ai